{
  "gene_name": "GTPase ERas",
  "gene": "UniProtKB:Q7Z444",
  "term_id": "GO:0007265",
  "gene_symbol": "ERAS",
  "term_label": "Ras protein signal transduction"
}